{
  "gene_name": "Late cornified envelope protein 5A",
  "term_label": "Unknown biological process",
  "gene": "UniProtKB:Q5TCM9",
  "term_id": "UNKNOWN:0002",
  "gene_symbol": "LCE5A"
}